{
  "term_id": "GO:0051959",
  "gene_name": "Rab-interacting lysosomal protein",
  "gene_symbol": "RILP",
  "term_label": "dynein light intermediate chain binding",
  "gene": "UniProtKB:Q96NA2"
}